{
  "gene_symbol": "SCGB1D2",
  "gene_name": "Secretoglobin family 1D member 2",
  "term_id": "UNKNOWN:0002",
  "gene": "UniProtKB:O95969",
  "term_label": "Unknown biological process"
}